{
  "term_label": "cytoplasm",
  "gene_symbol": "CSNK1A1",
  "gene": "UniProtKB:P48729",
  "gene_name": "Casein kinase I isoform alpha",
  "term_id": "GO:0005737"
}